{
  "gene_name": "Exosome complex component RRP42",
  "term_label": "nuclear exosome (RNase complex)",
  "gene_symbol": "EXOSC7",
  "gene": "UniProtKB:Q15024",
  "term_id": "GO:0000176"
}